{
  "gene_symbol": "ITPR3",
  "term_id": "GO:0070679",
  "term_label": "inositol 1,4,5 trisphosphate binding",
  "gene": "UniProtKB:Q14573",
  "gene_name": "Inositol 1,4,5-trisphosphate receptor type 3"
}